{
  "gene_name": "Protein SSX7",
  "gene": "UniProtKB:Q7RTT5",
  "term_id": "UNKNOWN:0002",
  "gene_symbol": "SSX7",
  "term_label": "Unknown biological process"
}